mesonephric tubule formation [GO:0072172] (biological process) Definition: The developmental process pertaining to the initial formation of a mesonephric tubule from unspecified parts. A mesonephric tubule is an epithelial tube that is part of the mesonephros. Relationships: is a type of nephron tubule formation [GO:0072079]; is part of mesonephric tubule morphogenesis [GO:0072171] Sources: GOC:mtg_kidney_jan10 Subtypes: ureteric bud formation [GO:0060676], GO:0061277, GO:0072181